alpha-galactosidase activity [GO:0004557] (molecular function) Subtypes: raffinose alpha-galactosidase activity [GO:0052692] Sources: EC:3.2.1.22 Also known as: melibiase activity, alpha-D-galactosidase activity Definition: Catalysis of the hydrolysis of terminal, non-reducing alpha-D-galactose residues in alpha-D-galactosides, including galactose oligosaccharides, galactomannans and galactolipids. Relationships: is a type of GO:0015925